{
  "term_id": "GO:0031410",
  "gene_symbol": "CAV1",
  "gene": "UniProtKB:Q03135",
  "term_label": "cytoplasmic vesicle",
  "gene_name": "Caveolin-1"
}